{
  "gene_name": "Proline-rich protein 30",
  "gene": "UniProtKB:Q53SZ7",
  "term_id": "UNKNOWN:0003",
  "term_label": "Unknown cellular component",
  "gene_symbol": "PRR30"
}